U4/U6 x U5 tri-snRNP complex [GO:0046540] (cellular component) Relationships: is a type of spliceosomal tri-snRNP complex [GO:0097526]; has part U5 snRNP [GO:0005682]; has part GO:0071001 Definition: A ribonucleoprotein complex that is formed by the association of the U4/U6 and U5 snRNPs. Also known as: U4/U6.U5 snRNP complex References: PMID:11867543 Sources: GOC:krc, GOC:pr, ISBN:0879695897